{
  "gene_symbol": "TIMM17B",
  "gene": "UniProtKB:O60830",
  "term_id": "GO:0030150",
  "term_label": "protein import into mitochondrial matrix",
  "gene_name": "Mitochondrial import inner membrane translocase subunit Tim17-B"
}